{
  "term_label": "Unknown cellular component",
  "term_id": "UNKNOWN:0003",
  "gene_symbol": "TNFRSF6B",
  "gene": "UniProtKB:O95407",
  "gene_name": "Tumor necrosis factor receptor superfamily member 6B"
}